{
  "term_id": "GO:0000786",
  "gene_symbol": "H2BC26",
  "gene": "UniProtKB:Q8N257",
  "term_label": "nucleosome",
  "gene_name": "Histone H2B type 3-B"
}